{
  "gene_symbol": "CKS2",
  "term_id": "GO:0043130",
  "term_label": "ubiquitin binding",
  "gene_name": "Cyclin-dependent kinases regulatory subunit 2",
  "gene": "UniProtKB:P33552"
}